{
  "gene": "UniProtKB:Q9Y5K8",
  "gene_symbol": "ATP6V1D",
  "gene_name": "V-type proton ATPase subunit D",
  "term_id": "GO:0033176",
  "term_label": "proton-transporting V-type ATPase complex"
}